{
  "term_label": "Unknown cellular component",
  "gene_symbol": "PTRH1",
  "term_id": "UNKNOWN:0003",
  "gene": "UniProtKB:Q86Y79",
  "gene_name": "Peptidyl-tRNA hydrolase"
}